{
  "term_id": "UNKNOWN:0001",
  "gene": "UniProtKB:Q86VY9",
  "gene_symbol": "TMEM200A",
  "gene_name": "Transmembrane protein 200A",
  "term_label": "Unknown molecular function"
}